{
  "term_label": "interleukin-5-mediated signaling pathway",
  "term_id": "GO:0038043",
  "gene": "UniProtKB:P05113",
  "gene_name": "Interleukin-5",
  "gene_symbol": "IL5"
}